{
  "gene_name": "Microcephalin",
  "term_id": "GO:0000278",
  "term_label": "mitotic cell cycle",
  "gene": "UniProtKB:Q8NEM0",
  "gene_symbol": "MCPH1"
}